ITP catabolic process [GO:0006193] (biological process) Definition: The chemical reactions and pathways resulting in the breakdown of ITP, inosine (5'-)triphosphate. Relationships: is a type of purine ribonucleotide catabolic process [GO:0009154]; is_a GO:0009207; is a type of ITP metabolic process [GO:0046041] Also known as: ITP breakdown, ITP catabolism, ITP degradation, ITP hydrolysis Sources: ISBN:0198506732